{
  "gene": "UniProtKB:O76024",
  "gene_name": "Wolframin",
  "gene_symbol": "WFS1",
  "term_label": "calcium ion homeostasis",
  "term_id": "GO:0055074"
}